{
  "gene_name": "Nucleoside diphosphate kinase B",
  "gene_symbol": "NME2",
  "gene": "UniProtKB:P22392",
  "term_id": "GO:0042981",
  "term_label": "regulation of apoptotic process"
}